{
  "gene_name": "Disintegrin and metalloproteinase domain-containing protein 19",
  "term_id": "GO:0006509",
  "term_label": "membrane protein ectodomain proteolysis",
  "gene_symbol": "ADAM19",
  "gene": "UniProtKB:Q9H013"
}